{
  "gene_symbol": "NSFL1C",
  "term_label": "autophagosome assembly",
  "term_id": "GO:0000045",
  "gene_name": "NSFL1 cofactor p47",
  "gene": "UniProtKB:Q9UNZ2"
}